{
  "term_id": "GO:0005737",
  "term_label": "cytoplasm",
  "gene_name": "RNA-binding protein Nova-2",
  "gene": "UniProtKB:Q9UNW9",
  "gene_symbol": "NOVA2"
}